asparagine transport [GO:0006867] (biological process) Definition: The directed movement of asparagine, alpha-aminosuccinamic acid, into, out of or within a cell, or between cells, by means of some agent such as a transporter or pore. Sources: GOC:ai Also known as: L-asparagine transport Relationships: is a type of GO:0015804; is a type of carboxylic acid transport [GO:0046942]; is a type of nitrogen compound transport [GO:0071705] Subtypes: L-asparagine import across plasma membrane [GO:1903811]